{
  "term_id": "GO:0019213",
  "gene_symbol": "NDST3",
  "gene": "UniProtKB:O95803",
  "gene_name": "Bifunctional heparan sulfate N-deacetylase_N-sulfotransferase 3",
  "term_label": "deacetylase activity"
}